{
  "term_label": "Golgi-associated vesicle",
  "term_id": "GO:0005798",
  "gene_symbol": "MAP6D1",
  "gene_name": "MAP6 domain-containing protein 1",
  "gene": "UniProtKB:Q9H9H5"
}